{
  "gene_symbol": "IGHV3-15",
  "gene_name": "Immunoglobulin heavy variable 3-15",
  "gene": "UniProtKB:A0A0B4J1V0",
  "term_label": "antigen binding",
  "term_id": "GO:0003823"
}